cardiac muscle cell myoblast differentiation [GO:0060379] (biological process) Definition: The process in which a relatively unspecialized cell acquires specialized features of a cardiac myoblast. A cardiac myoblast is a precursor cell that has been committed to a cardiac muscle cell fate but retains the ability to divide and proliferate throughout life. Also known as: myocardial precursor cell differentiation, cardiac myoblast differentiation Regulation: regulated by regulation of cardiac muscle cell myoblast differentiation [GO:2000690]; negatively regulated by negative regulation of cardiac muscle cell myoblast differentiation [GO:2000691]; positively regulated by positive regulation of cardiac muscle cell myoblast differentiation [GO:2000700] Relationships: is a type of GO:0010002; is a type of GO:0045445 Sources: GOC:dph, GOC:tb